nitric oxide transport [GO:0030185] (BP) Relationships: is a type of nitrogen compound transport [GO:0071705] Sources: GOC:mah Definition: The directed movement of nitric oxide, nitrogen monoxide, into, out of or within a cell, or between cells, by means of some agent such as a transporter or pore.